{
  "term_id": "GO:0008283",
  "gene_name": "Ankyrin repeat domain-containing protein 45",
  "gene": "UniProtKB:Q5TZF3",
  "term_label": "cell population proliferation",
  "gene_symbol": "ANKRD45"
}